{
  "gene_symbol": "CLBA1",
  "gene": "UniProtKB:Q96F83",
  "gene_name": "Uncharacterized protein CLBA1",
  "term_id": "UNKNOWN:0002",
  "term_label": "Unknown biological process"
}